{
  "gene_symbol": "GOLGA8K",
  "term_id": "GO:0000137",
  "term_label": "Golgi cis cisterna",
  "gene": "UniProtKB:D6RF30",
  "gene_name": "Golgin subfamily A member 8K"
}